{
  "gene_name": "Putative uncharacterized protein encoded by LINC01553",
  "term_id": "UNKNOWN:0003",
  "term_label": "Unknown cellular component",
  "gene": "UniProtKB:A4QN01",
  "gene_symbol": "LINC01553"
}